regulation of amino acid metabolic process [GO:0006521] (biological process) Also known as: regulation of amino acid metabolism Definition: Any process that modulates the frequency, rate or extent of the chemical reactions and pathways involving amino acids. Sources: GOC:go_curators Subtypes: regulation of 1-aminocyclopropane-1-carboxylate metabolic process [GO:0010602], negative regulation of amino acid metabolic process [GO:0045763], positive regulation of amino acid metabolic process [GO:0045764], GO:0090357, regulation of ornithine metabolic process [GO:0090368], regulation of arginine catabolic process [GO:1900081], GO:1901413, GO:1901494, GO:1901715, regulation of glutamate metabolic process [GO:2000211], regulation of L-proline metabolic process [GO:2000214], regulation of amino acid biosynthetic process [GO:2000282] Relationships: is a type of regulation of primary metabolic process [GO:0080090]; regulates amino acid metabolic process [GO:0006520]